{
  "gene": "UniProtKB:P15311",
  "gene_symbol": "EZR",
  "gene_name": "Ezrin",
  "term_id": "GO:0005886",
  "term_label": "plasma membrane"
}